{
  "gene_symbol": "ELL2",
  "gene_name": "RNA polymerase II elongation factor ELL2",
  "term_id": "GO:0000987",
  "term_label": "cis-regulatory region sequence-specific DNA binding",
  "gene": "UniProtKB:O00472"
}